{
  "gene": "UniProtKB:Q6XUX3",
  "term_id": "GO:0070374",
  "term_label": "positive regulation of ERK1 and ERK2 cascade",
  "gene_name": "Dual serine_threonine and tyrosine protein kinase",
  "gene_symbol": "DSTYK"
}